{
  "gene_name": "PiggyBac transposable element-derived protein 4",
  "gene_symbol": "PGBD4",
  "term_id": "UNKNOWN:0002",
  "gene": "UniProtKB:Q96DM1",
  "term_label": "Unknown biological process"
}